positive regulation of JUN kinase activity [GO:0043507] (BP) Definition: Any process that activates or increases the frequency, rate or extent of JUN kinase activity. Sources: GOC:jl Also known as: positive regulation of JUNK activity, up regulation of JNK activity, up-regulation of JNK activity, upregulation of JNK activity, stimulation of JNK activity Relationships: is a type of GO:0043406; is a type of regulation of JUN kinase activity [GO:0043506]; positively regulates JUN kinase activity [GO:0004705]